{
  "gene": "UniProtKB:Q9H9Y2",
  "gene_name": "Ribosome production factor 1",
  "gene_symbol": "RPF1",
  "term_id": "GO:0030687",
  "term_label": "preribosome, large subunit precursor"
}